{
  "term_label": "RNA binding",
  "gene_name": "Small ribosomal subunit protein eS19",
  "term_id": "GO:0003723",
  "gene_symbol": "RPS19",
  "gene": "UniProtKB:P39019"
}